glycoside catabolic process [GO:0016139] (biological process) Sources: GOC:go_curators Subtypes: saponin catabolic process [GO:0016136], GO:0019391, aminoglycoside antibiotic catabolic process [GO:0030649], cyanogenic glycoside catabolic process [GO:0042342], GO:0046284, GO:1901120, butirosin catabolic process [GO:1901757], GO:1901805 Also known as: O-glycoside breakdown, O-glycoside catabolic process, O-glycoside catabolism, O-glycoside degradation, glycoside breakdown, glycoside catabolism, glycoside degradation Definition: The chemical reactions and pathways resulting in the breakdown of glycosides, compounds in which a glycosyl group is substituted into a hydroxyl, thiol or selenol group in another compound. Relationships: is a type of glycoside metabolic process [GO:0016137]; is a type of glycosyl compound catabolic process [GO:1901658]